{
  "gene": "UniProtKB:Q9UF33",
  "term_id": "GO:0007411",
  "gene_name": "Ephrin type-A receptor 6",
  "gene_symbol": "EPHA6",
  "term_label": "axon guidance"
}